{
  "term_label": "neuron projection",
  "gene_symbol": "RGS7BP",
  "gene_name": "Regulator of G-protein signaling 7-binding protein",
  "gene": "UniProtKB:Q6MZT1",
  "term_id": "GO:0043005"
}